positive regulation of protection from non-homologous end joining at telomere [GO:1905766] (biological process) Definition: Any process that activates or increases the frequency, rate or extent of protection from non-homologous end joining at telomere. References: PMID:14690602 Sources: GOC:BHF, GOC:BHF_telomere, GOC:TermGenie, GOC:nc, GO_REF:0000058 Also known as: positive regulation of protection from NHEJ-mediated telomere fusion, up regulation of protection from NHEJ-mediated telomere fusion, up regulation of protection from non-homologous end joining at telomere, up-regulation of protection from NHEJ-mediated telomere fusion, up-regulation of protection from non-homologous end joining at telomere, upregulation of protection from NHEJ-mediated telomere fusion, upregulation of protection from non-homologous end joining at telomere, activation of protection from NHEJ-mediated telomere fusion, activation of protection from non-homologous end joining at telomere Relationships: is_a positive regulation of telomere maintenance in response to DNA damage [GO:1904507]; is a type of GO:1905764; RO_0002213 protection from non-homologous end joining at telomere [GO:0031848]